prenyl diphosphate synthase activity [GO:0120531] (molecular function) Relationships: is a type of GO:0004659 Also known as: IPPS activity, isoprenyl pyrophosphate synthase activity Definition: Catalysis of chain elongation of prenyl diphosphate substrates via one or more condensation reactions with isopentenyl diphosphate to generate linear polymers with defined chain lengths. Subtypes: heptaprenyl diphosphate synthase activity [GO:0000010], dimethylallyltranstransferase activity [GO:0004161], geranylgeranyl diphosphate synthase activity [GO:0004311], (2E,6E)-farnesyl diphosphate synthase activity [GO:0004337], hexaprenyl-diphosphate synthase ((2E,6E)-farnesyl-diphosphate specific) activity [GO:0036423], GO:0044687, ditrans,polycis-polyprenyl diphosphate synthase [(2E,6E)-farnesyl diphosphate specific] activity [GO:0045547], dimethylallylcistransferase activity [GO:0047863], GO:0050267, hexaprenyl diphosphate synthase (geranylgeranyl-diphosphate specific) activity [GO:0052922], all-trans-nonaprenyl-diphosphate synthase (geranyl-diphosphate specific) activity [GO:0052923], all-trans-nonaprenyl-diphosphate synthase (geranylgeranyl-diphosphate specific) activity [GO:0052924], GO:0097269, GO:0102059, all-trans-octaprenyl-diphosphate synthase activity [GO:0106350] References: PMID:12135472, PMID:26216239